{
  "term_id": "UNKNOWN:0002",
  "gene_symbol": "B3GNTL1",
  "gene": "UniProtKB:Q67FW5",
  "gene_name": "UDP-GlcNAc:betaGal beta-1,3-N-acetylglucosaminyltransferase-like protein 1",
  "term_label": "Unknown biological process"
}